NAD(P)H oxidase H2O2-forming activity [GO:0016174] (molecular function) References: PMID:10401672, PMID:10601291, PMID:11822874 Sources: EC:1.6.3.1 Definition: Catalysis of the reaction: NAD(P)H + H+ + O2 = NAD(P)+ + hydrogen peroxide. Relationships: is a type of oxidoreductase activity, acting on NAD(P)H, oxygen as acceptor [GO:0050664] Regulation: positively regulated by positive regulation of NAD(P)H oxidase activity [GO:0033864] Also known as: NAD(P)H oxidase activity, NADPH oxidase, THOX2 activity, ThOX activity, thyroid NADPH oxidase activity, thyroid oxidase 2 activity, thyroid oxidase activity, NAD(P)H:oxygen oxidoreductase activity, dual oxidase activity, p138tox